{
  "term_id": "GO:0030906",
  "term_label": "retromer, cargo-selective complex",
  "gene_name": "Vacuolar protein sorting-associated protein 26A",
  "gene_symbol": "VPS26A",
  "gene": "UniProtKB:O75436"
}